{
  "gene": "UniProtKB:P0DMP2",
  "term_label": "glutamatergic synapse",
  "term_id": "GO:0098978",
  "gene_name": "SLIT-ROBO Rho GTPase-activating protein 2B",
  "gene_symbol": "SRGAP2B"
}